{
  "term_id": "UNKNOWN:0002",
  "gene_symbol": "CDK11A",
  "gene": "UniProtKB:Q9UQ88",
  "gene_name": "Cyclin-dependent kinase 11A",
  "term_label": "Unknown biological process"
}